3-hydroxybutyrate dehydrogenase activity [GO:0003858] (molecular function) Definition: Catalysis of the reaction: (R)-3-hydroxybutanoate + NAD+ = acetoacetate + H+ + NADH. Also known as: D-beta-hydroxybutyrate dehydrogenase activity Sources: EC:1.1.1.30, RHEA:20521 Relationships: is a type of GO:0016616